cardiac septum development [GO:0003279] (biological process) Relationships: is a type of GO:0048856; BFO_0000050 cardiac chamber development [GO:0003205] Sources: GOC:mtg_heart Also known as: heart septum development Subtypes: GO:0003281, atrial septum development [GO:0003283] Definition: The progression of a cardiac septum over time, from its initial formation to the mature structure.